{
  "term_id": "GO:0042594",
  "gene_symbol": "PCK1",
  "gene_name": "Phosphoenolpyruvate carboxykinase, cytosolic [GTP]",
  "term_label": "response to starvation",
  "gene": "UniProtKB:P35558"
}